{
  "gene_name": "AMP deaminase 2",
  "gene": "UniProtKB:Q01433",
  "gene_symbol": "AMPD2",
  "term_id": "GO:0046033",
  "term_label": "AMP metabolic process"
}